protein propionyltransferase activity [GO:0061920] (molecular function) Definition: Catalysis of the reaction: propionyl-CoA + lysine in peptide = CoA + N-propionyl-lysine-peptide. References: PMID:17267393 Relationships: is a type of N-acyltransferase activity [GO:0016410] Subtypes: histone propionyltransferase activity [GO:0061922]